{
  "term_label": "plasma membrane",
  "gene_symbol": "OR52E6",
  "gene_name": "Olfactory receptor 52E6",
  "gene": "UniProtKB:Q96RD3",
  "term_id": "GO:0005886"
}